{
  "gene": "UniProtKB:Q96HA1",
  "term_id": "GO:0006405",
  "gene_name": "Nuclear envelope pore membrane protein POM 121",
  "term_label": "RNA export from nucleus",
  "gene_symbol": "POM121"
}